{
  "gene_name": "MaFF-interacting protein",
  "gene_symbol": "MAFIP",
  "term_id": "UNKNOWN:0003",
  "term_label": "Unknown cellular component",
  "gene": "UniProtKB:Q8WZ33"
}